{
  "gene_name": "Kinesin-like protein KIF3B",
  "term_id": "GO:0005737",
  "gene": "UniProtKB:O15066",
  "term_label": "cytoplasm",
  "gene_symbol": "KIF3B"
}